{
  "term_id": "GO:0000209",
  "term_label": "protein polyubiquitination",
  "gene": "UniProtKB:P62256",
  "gene_name": "Ubiquitin-conjugating enzyme E2 H",
  "gene_symbol": "UBE2H"
}